{
  "gene": "UniProtKB:Q99880",
  "term_id": "GO:0019731",
  "gene_name": "Histone H2B type 1-L",
  "gene_symbol": "H2BC13",
  "term_label": "antibacterial humoral response"
}